{
  "gene": "UniProtKB:P11177",
  "term_id": "GO:0045254",
  "gene_symbol": "PDHB",
  "term_label": "pyruvate dehydrogenase complex",
  "gene_name": "Pyruvate dehydrogenase E1 component subunit beta, mitochondrial"
}